{
  "term_id": "GO:0005634",
  "gene": "UniProtKB:P49750",
  "gene_symbol": "YLPM1",
  "gene_name": "YLP motif-containing protein 1",
  "term_label": "nucleus"
}